{
  "gene_symbol": "LOC730098",
  "gene": "UniProtKB:G3V523",
  "term_id": "UNKNOWN:0001",
  "gene_name": "HCG2040265, isoform CRA_a",
  "term_label": "Unknown molecular function"
}